{
  "gene_name": "Immunoglobulin heavy variable 3-9",
  "gene_symbol": "IGHV3-9",
  "term_id": "GO:0016064",
  "term_label": "immunoglobulin mediated immune response",
  "gene": "UniProtKB:P01782"
}